negative regulation of ethylene biosynthetic process [GO:0010366] (biological process) Definition: Any process that stops, prevents, or reduces the frequency, rate or extent of an ethylene biosynthetic process. Sources: GOC:tair_curators Relationships: is a type of regulation of ethylene biosynthetic process [GO:0010364]; is a type of GO:1900912; negatively regulates ethylene biosynthetic process [GO:0009693]